{
  "term_id": "GO:0003725",
  "gene_symbol": "SIDT1",
  "gene_name": "SID1 transmembrane family member 1",
  "term_label": "double-stranded RNA binding",
  "gene": "UniProtKB:Q9NXL6"
}